{
  "term_label": "U4/U6 x U5 tri-snRNP complex",
  "gene": "UniProtKB:P62312",
  "gene_symbol": "LSM6",
  "term_id": "GO:0046540",
  "gene_name": "U6 snRNA-associated Sm-like protein LSm6"
}